{
  "gene": "UniProtKB:P68366",
  "gene_name": "Tubulin alpha-4A chain",
  "term_id": "GO:0030182",
  "gene_symbol": "TUBA4A",
  "term_label": "neuron differentiation"
}